{
  "term_label": "DNA binding",
  "term_id": "GO:0003677",
  "gene_name": "Histone H2B type 3-B",
  "gene": "UniProtKB:Q8N257",
  "gene_symbol": "H2BC26"
}